horizontal cell localization [GO:0035852] (biological process) Definition: Any process in which a horizontal cell is transported to, and/or maintained in, a specific location within the inner nuclear layer (INL) of the retina. A horizontal cell is a neuron that laterally connects other neurons in the inner nuclear layer (INL) of the retina. Targeting of retinal neurons to the appropriate lamina is vital to establish the architecture of the retina. References: PMID:18094249 Sources: CL:0000745, GOC:bf, GOC:yaf Also known as: horizontal cell localisation, horizontal cell positioning, laminar positioning of retinal horizontal cell, retinal horizontal cell positioning Relationships: is a type of GO:0051674; is part of retina layer formation [GO:0010842] Regulation: regulated by regulation of horizontal cell localization [GO:1902872]; negatively regulated by negative regulation of horizontal cell localization [GO:1902873]; positively regulated by positive regulation of horizontal cell localization [GO:1902874]